{
  "gene": "UniProtKB:Q6B0K9",
  "term_label": "oxygen carrier activity",
  "gene_symbol": "HBM",
  "gene_name": "Hemoglobin subunit mu",
  "term_id": "GO:0005344"
}